receptor-mediated bacteriophage irreversible attachment to host cell [GO:0098002] (biological process) Definition: The processes by which a bacteriophage initially commits to infection by binding the host receptor irreversibly. Disruption of the phage:cell complex at this step results in the loss of infective phage virions since the process is characterized by conformational changes of bacteriophage head and tail proteins and injection of bacteriophage proteins into the infected cell. Sources: GOC:bm Also known as: irreversible bacteriophage attachment, binding of host cell surface receptor, phage irreversible adsorption Relationships: is_a entry receptor-mediated virion attachment to host cell [GO:0098670]